{
  "gene_name": "Ankyrin repeat domain-containing protein 53",
  "gene_symbol": "ANKRD53",
  "term_label": "positive regulation of microtubule polymerization",
  "term_id": "GO:0031116",
  "gene": "UniProtKB:Q8N9V6"
}